positive regulation of cellooligosaccharide catabolic process [GO:2000965] (biological process) Sources: GOC:mengo_curators Relationships: is a type of positive regulation of catabolic process [GO:0009896]; is a type of positive regulation of carbohydrate metabolic process [GO:0045913]; is_a regulation of cellooligosaccharide catabolic process [GO:2000963]; positively regulates cellooligosaccharide catabolic process [GO:2000903] Definition: Any process that activates or increases the frequency, rate or extent of cellooligosaccharide catabolic process. Also known as: positive regulation of cellooligosaccharide catabolism